pyrophosphatase activity [GO:0016462] (molecular function) Definition: Catalysis of the hydrolysis of a pyrophosphate bond (diphosphate bond) between two phosphate groups. Sources: GOC:curators, https://en.wikipedia.org/wiki/Pyrophosphatase Relationships: is a type of GO:0016818 Subtypes: endopolyphosphatase activity [GO:0000298], GO:0000810, 4-amino-5-hydroxymethyl-2-methylpyrimidine diphosphatase activity [GO:0002145], GO:0003998, apyrase activity [GO:0004050], exopolyphosphatase activity [GO:0004309], inorganic diphosphate phosphatase activity [GO:0004427], dinucleotide phosphatase activity [GO:0004551], GO:0004636, GO:0004787, GO:0008486, CDP-diacylglycerol diphosphatase activity [GO:0008715], UDP-2,3-diacylglucosamine hydrolase activity [GO:0008758], GO:0008768, bis(5'-nucleosyl)-tetraphosphatase activity [GO:0008796], GO:0008894, GO:0010945, GO:0017110, ribonucleoside triphosphate phosphatase activity [GO:0017111], ADP-sugar diphosphatase activity [GO:0019144], dihydroneopterin triphosphate pyrophosphohydrolase activity [GO:0019177], GO:0033699, mRNA 5'-diphosphatase activity [GO:0034353], bis(5'-adenosyl)-hexaphosphatase activity [GO:0034431], bis(5'-adenosyl)-pentaphosphatase activity [GO:0034432], 5-phosphoribosyl 1-pyrophosphate pyrophosphatase activity [GO:0043135], GO:0047429, oligosaccharide-diphosphodolichol diphosphatase activity [GO:0047430], adenosine-tetraphosphatase activity [GO:0047624], ADP-ribose diphosphatase activity [GO:0047631], bis(5'-adenosyl)-triphosphatase activity [GO:0047710], GO:0047734, thiamine triphosphate phosphatase activity [GO:0050333], inorganic triphosphate phosphatase activity [GO:0050355], GO:0052751, isoprenoid diphosphate phosphatase activity [GO:0106405], RNA NAD-cap (NMN-forming) hydrolase activity [GO:0110153], DNA-3'-diphospho-5'-guanosine diphosphatase activity [GO:0120108], all-trans-phytoene synthase activity [GO:0140630], mRNA 5'-triphosphate monophosphatase activity [GO:0140818], 5'-(N(7)-methyl 5'-triphosphoguanosine)-[mRNA] diphosphatase activity [GO:0140932], 5'-(N(7)-methylguanosine 5'-triphospho)-[mRNA] hydrolase activity [GO:0140933]